negative regulation of glycoprotein biosynthetic process [GO:0010561] (biological process) Definition: Any process that decreases the rate, frequency, or extent of the chemical reactions and pathways resulting in the formation of a glycoprotein, a protein that contains covalently bound glycose (i.e. monosaccharide) residues; the glycose occurs most commonly as oligosaccharide or fairly small polysaccharide but occasionally as monosaccharide. Sources: GOC:dph, GOC:tb Relationships: is a type of negative regulation of macromolecule biosynthetic process [GO:0010558]; is a type of regulation of glycoprotein biosynthetic process [GO:0010559]; is a type of negative regulation of glycoprotein metabolic process [GO:1903019]; negatively regulates glycoprotein biosynthetic process [GO:0009101] Subtypes: negative regulation of amyloid precursor protein biosynthetic process [GO:0042985], negative regulation of proteoglycan biosynthetic process [GO:1902729], negative regulation of protein O-linked glycosylation [GO:1904099]